prepulse inhibition [GO:0060134] (biological process) Definition: The process in which a startle magnitude is reduced when the startling stimulus is preceded by a low-intensity prepulse. Relationships: is a type of negative regulation of response to external stimulus [GO:0032102]; is part of startle response [GO:0001964] References: PMID:10341260 Sources: GOC:dph Also known as: pre-pulse inhibition, PPI